{
  "gene_symbol": "GNAS",
  "term_id": "GO:0051430",
  "gene": "UniProtKB:Q5JWF2",
  "term_label": "corticotropin-releasing hormone receptor 1 binding",
  "gene_name": "Guanine nucleotide-binding protein G(s) subunit alpha isoforms XLas"
}